pyridoxal biosynthetic process [GO:0042821] (biological process) Also known as: pyridoxal anabolism, pyridoxal biosynthesis, pyridoxal formation, pyridoxal synthesis References: PMID:21767669 Sources: GOC:jl Relationships: is a type of pyridoxal metabolic process [GO:0042817]; is a type of vitamin B6 biosynthetic process [GO:0042819]; is a type of aldehyde biosynthetic process [GO:0046184] Definition: The chemical reactions and pathways resulting in the formation of 3-hydroxy-5-(hydroxymethyl)-2-methyl-4-pyridinecarboxaldehyde, one of the vitamin B6 compounds.